{
  "gene": "UniProtKB:B2RUY7",
  "term_id": "GO:0032281",
  "gene_symbol": "VWC2L",
  "term_label": "AMPA glutamate receptor complex",
  "gene_name": "von Willebrand factor C domain-containing protein 2-like"
}